{
  "gene": "UniProtKB:Q8N6M6",
  "gene_symbol": "AOPEP",
  "term_id": "UNKNOWN:0002",
  "gene_name": "Aminopeptidase O",
  "term_label": "Unknown biological process"
}